negative regulation of cellular response to hepatocyte growth factor stimulus [GO:2001113] (biological process) Definition: Any process that stops, prevents or reduces the frequency, rate or extent of cellular response to hepatocyte growth factor stimulus. Also known as: negative regulation of cellular response to HGF stimulus Sources: GOC:obol Relationships: is a type of negative regulation of cellular response to growth factor stimulus [GO:0090288]; is a type of regulation of cellular response to hepatocyte growth factor stimulus [GO:2001112]; RO_0002212 cellular response to hepatocyte growth factor stimulus [GO:0035729]